{
  "gene_name": "Serine_threonine-protein kinase H2",
  "gene_symbol": "PSKH2",
  "gene": "UniProtKB:Q96QS6",
  "term_label": "protein serine/threonine kinase activity",
  "term_id": "GO:0004674"
}